{
  "term_id": "UNKNOWN:0003",
  "gene_symbol": "CTSL3P",
  "gene": "UniProtKB:Q5NE16",
  "term_label": "Unknown cellular component",
  "gene_name": "Putative inactive cathepsin L-like protein CTSL3P"
}